{
  "term_id": "UNKNOWN:0001",
  "term_label": "Unknown molecular function",
  "gene_symbol": "TMEM19",
  "gene": "UniProtKB:Q96HH6",
  "gene_name": "Transmembrane protein 19"
}